{
  "term_id": "GO:0005789",
  "term_label": "endoplasmic reticulum membrane",
  "gene_symbol": "JAGN1",
  "gene": "UniProtKB:Q8N5M9",
  "gene_name": "Protein jagunal homolog 1"
}